{
  "term_label": "Unknown molecular function",
  "term_id": "UNKNOWN:0001",
  "gene_symbol": "PHF14",
  "gene_name": "PHD finger protein 14",
  "gene": "UniProtKB:O94880"
}